{
  "term_label": "mitochondrial electron transport, succinate to ubiquinone",
  "gene_name": "Succinate dehydrogenase cytochrome b560 subunit, mitochondrial",
  "term_id": "GO:0006121",
  "gene_symbol": "SDHC",
  "gene": "UniProtKB:Q99643"
}